{
  "term_label": "Unknown biological process",
  "term_id": "UNKNOWN:0002",
  "gene": "UniProtKB:Q8TC84",
  "gene_name": "Fibronectin type 3 and ankyrin repeat domains protein 1",
  "gene_symbol": "FANK1"
}